{
  "gene_name": "Threonine synthase-like 2",
  "term_id": "UNKNOWN:0003",
  "gene": "UniProtKB:Q86YJ6",
  "term_label": "Unknown cellular component",
  "gene_symbol": "THNSL2"
}